{
  "gene": "UniProtKB:P0DP24",
  "gene_symbol": "CALM2",
  "gene_name": "Calmodulin-2",
  "term_label": "nucleus",
  "term_id": "GO:0005634"
}